{
  "term_id": "GO:0005587",
  "gene": "UniProtKB:Q14031",
  "term_label": "collagen type IV trimer",
  "gene_symbol": "COL4A6",
  "gene_name": "Collagen alpha-6(IV) chain"
}